{
  "term_label": "phosphorylase kinase complex",
  "gene_name": "Phosphorylase b kinase regulatory subunit alpha, skeletal muscle isoform",
  "gene_symbol": "PHKA1",
  "gene": "UniProtKB:P46020",
  "term_id": "GO:0005964"
}